damaged DNA binding [GO:0003684] (molecular function) Definition: Binding to damaged DNA. Subtypes: alkylated DNA binding [GO:0032131], oxidized DNA binding [GO:0032356], DNA-(abasic site) binding [GO:0140431], single-strand break-containing DNA binding [GO:1990165] Sources: GOC:jl Also known as: DNA repair enzyme, DNA repair protein Relationships: is a type of DNA binding [GO:0003677]